{
  "gene_symbol": "EPPK1",
  "term_id": "GO:0042060",
  "term_label": "wound healing",
  "gene": "UniProtKB:P58107",
  "gene_name": "Epiplakin"
}